{
  "term_id": "GO:1902514",
  "gene_name": "Voltage-dependent calcium channel gamma-6 subunit",
  "gene": "UniProtKB:Q9BXT2",
  "term_label": "regulation of calcium ion transmembrane transport via high voltage-gated calcium channel",
  "gene_symbol": "CACNG6"
}